ornithine carbamoyltransferase activity [GO:0004585] (molecular function) Regulation: negatively regulated by ornithine carbamoyltransferase inhibitor activity [GO:0090369] Relationships: is a type of GO:0016743; is part of ornithine metabolic process [GO:0006591] Also known as: L-ornithine carbamoyltransferase activity, L-ornithine carbamyltransferase activity, L-ornithine transcarbamylase activity, OTC activity, OTCase activity, carbamoyl-phosphate:L-ornithine carbamoyltransferase activity, carbamylphosphate-ornithine transcarbamylase activity, citrulline phosphorylase activity, ornithine carbamyltransferase activity, ornithine transcarbamylase activity Sources: EC:2.1.3.3 Definition: Catalysis of the reaction: carbamoyl phosphate + L-ornithine = phosphate + L-citrulline.